{
  "gene": "UniProtKB:Q5VWK5",
  "term_id": "GO:0009897",
  "gene_name": "Interleukin-23 receptor",
  "gene_symbol": "IL23R",
  "term_label": "external side of plasma membrane"
}